neuron migration [GO:0001764] (biological process) Sources: CL:0000540, GOC:go_curators Also known as: neuron chemotaxis, neuronal migration, neuron guidance Subtypes: neuron migration involved in retrograde extension [GO:0003393], gonadotrophin-releasing hormone neuronal migration to the hypothalamus [GO:0021828], outward migration of deep nuclear neurons [GO:0021947], inward migration of deep nuclear neurons [GO:0021948], motor neuron migration [GO:0097475], GO:0140650, GO:1904936, GO:1904937 Regulation: regulated by regulation of neuron migration [GO:2001222]; negatively regulated by negative regulation of neuron migration [GO:2001223]; positively regulated by positive regulation of neuron migration [GO:2001224] Definition: The characteristic movement of an immature neuron from germinal zones to specific positions where they will reside as they mature. Relationships: is a type of cell migration [GO:0016477]; is part of generation of neurons [GO:0048699]